regulation of granulosa cell proliferation [GO:1904195] (biological process) Definition: Any process that modulates the frequency, rate or extent of granulosa cell proliferation. Relationships: is_a regulation of epithelial cell proliferation [GO:0050678]; regulates GO:1990739 References: PMID:22383759 Sources: GOC:TermGenie, GO_REF:0000058 Subtypes: negative regulation of granulosa cell proliferation [GO:1904196], positive regulation of granulosa cell proliferation [GO:1904197]